{
  "gene_symbol": "AADACL4",
  "term_label": "Unknown molecular function",
  "term_id": "UNKNOWN:0001",
  "gene_name": "Arylacetamide deacetylase-like 4",
  "gene": "UniProtKB:Q5VUY2"
}